{
  "gene_symbol": "FLT1",
  "gene": "UniProtKB:P17948",
  "term_id": "GO:0019838",
  "gene_name": "Vascular endothelial growth factor receptor 1",
  "term_label": "growth factor binding"
}